{
  "gene": "UniProtKB:O95409",
  "gene_name": "Zinc finger protein ZIC 2",
  "term_label": "regulation of transcription by RNA polymerase II",
  "term_id": "GO:0006357",
  "gene_symbol": "ZIC2"
}